{
  "gene": "UniProtKB:A4D1T9",
  "gene_name": "Probable inactive serine protease 37",
  "term_id": "GO:0051604",
  "term_label": "protein maturation",
  "gene_symbol": "PRSS37"
}